SMN-Gemin2 complex [GO:0034718] (cellular component) References: PMID:17640873 Sources: GOC:mah Definition: A protein complex that contains the survival motor neuron (SMN) protein and Gemin2; may form the stable core of the larger SMN complex. Relationships: is a type of GO:0090575; is a type of Sm-like protein family complex [GO:0120114]